{
  "term_label": "cytoplasm",
  "gene": "UniProtKB:Q9UK97",
  "gene_symbol": "FBXO9",
  "term_id": "GO:0005737",
  "gene_name": "F-box only protein 9"
}